{
  "term_label": "immune response",
  "gene_name": "Interleukin-36 gamma",
  "gene": "UniProtKB:Q9NZH8",
  "gene_symbol": "IL36G",
  "term_id": "GO:0006955"
}